{
  "term_id": "GO:0046847",
  "gene_name": "Spermatogenesis-associated protein 13",
  "term_label": "filopodium assembly",
  "gene_symbol": "SPATA13",
  "gene": "UniProtKB:Q96N96"
}